{
  "gene_name": "Major intrinsically disordered Notch2-binding receptor 1",
  "term_id": "GO:0005886",
  "gene_symbol": "MINAR1",
  "term_label": "plasma membrane",
  "gene": "UniProtKB:Q9UPX6"
}